{
  "gene_name": "Large ribosomal subunit protein uL13m",
  "gene": "UniProtKB:Q9BYD1",
  "term_label": "mRNA binding",
  "gene_symbol": "MRPL13",
  "term_id": "GO:0003729"
}